{
  "gene": "UniProtKB:Q5TA81",
  "term_id": "UNKNOWN:0003",
  "term_label": "Unknown cellular component",
  "gene_name": "Late cornified envelope protein 2C",
  "gene_symbol": "LCE2C"
}